{
  "gene_name": "Deleted in azoospermia protein 2",
  "term_id": "GO:0045948",
  "gene_symbol": "DAZ2",
  "term_label": "positive regulation of translational initiation",
  "gene": "UniProtKB:Q13117"
}